CUC codon-amino acid adaptor activity [GO:0033418] (molecular function) Note: Note that in the standard genetic code, CTC codes for leucine. Definition: A triplet codon-amino acid adaptor activity that recognizes a CUC codon. Also known as: CTC codon-amino acid adaptor activity, leucine tRNA Sources: GOC:mah Relationships: is a type of triplet codon-amino acid adaptor activity [GO:0030533]